{
  "gene_symbol": "FOXD4L1",
  "term_id": "GO:0030154",
  "gene_name": "Forkhead box protein D4-like 1",
  "term_label": "cell differentiation",
  "gene": "UniProtKB:Q9NU39"
}